chemotaxis to oxidizable substrate [GO:0042333] (biological process) References: PMID:11029423 Sources: GOC:jl Definition: The directed movement of a motile cell or organism in response to the presence of an oxidizable substrate, for example, fructose. Relationships: is a type of chemotaxis [GO:0006935]; is a type of energy taxis [GO:0009453] Also known as: taxis in response to oxidizable substrate